{
  "gene_symbol": "RTL9",
  "gene_name": "Retrotransposon Gag-like protein 9",
  "term_id": "UNKNOWN:0002",
  "term_label": "Unknown biological process",
  "gene": "UniProtKB:Q8NET4"
}